neuromuscular junction of somatic muscle [GO:0098527] (cellular component) Relationships: is a type of GO:0031594 Subtypes: GO:0098524 Definition: A neuromuscular junction in which the target muscle cell is a somatic muscle cell, such as those found in nematodes and arthropods. Sources: GOC:dos